{
  "gene_symbol": "ATP8B3",
  "term_label": "Golgi organization",
  "gene_name": "Phospholipid-transporting ATPase IK",
  "term_id": "GO:0007030",
  "gene": "UniProtKB:O60423"
}